{
  "gene_symbol": "TSPYL1",
  "term_id": "GO:0042393",
  "gene_name": "Testis-specific Y-encoded-like protein 1",
  "gene": "UniProtKB:Q9H0U9",
  "term_label": "histone binding"
}